lysosomal lumen [GO:0043202] (CC) Relationships: is a type of vacuolar lumen [GO:0005775]; is part of lysosome [GO:0005764] Subtypes: endolysosome lumen [GO:0036021], acrosomal lumen [GO:0043160] Definition: The volume enclosed within the lysosomal membrane. References: PMID:15213228 Sources: GOC:jl